{
  "gene_name": "Protein phosphatase 1 regulatory subunit 26",
  "gene_symbol": "PPP1R26",
  "term_id": "UNKNOWN:0001",
  "term_label": "Unknown molecular function",
  "gene": "UniProtKB:Q5T8A7"
}